Kv4.3-DPP6 channel complex [GO:0071201] (cellular component) References: PMID:12575952, PMID:15911355 Definition: A voltage-gated potassium channel complex that contains the peptidase-related protein DPP6 associated with the channel via interaction with the Kv alpha subunit 4.3. Also known as: Kv4.3-DPPX channel complex Relationships: is a type of voltage-gated potassium channel complex [GO:0008076]